positive regulation of androgen receptor signaling pathway [GO:0160207] (biological process) Relationships: is a type of positive regulation of intracellular steroid hormone receptor signaling pathway [GO:0033145]; is a type of regulation of androgen receptor signaling pathway [GO:0060765]; positively regulates androgen receptor signaling pathway [GO:0030521] References: PMID:29057879 Definition: Any process that activates or increases the frequency, rate or extent of androgen receptor signaling.